{
  "term_label": "membrane",
  "gene_name": "Golgi-associated PDZ and coiled-coil motif-containing protein",
  "term_id": "GO:0016020",
  "gene_symbol": "GOPC",
  "gene": "UniProtKB:Q9HD26"
}